{
  "gene_name": "Peroxisome biogenesis factor 2",
  "gene": "UniProtKB:P28328",
  "gene_symbol": "PEX2",
  "term_label": "Cdc73/Paf1 complex",
  "term_id": "GO:0016593"
}